tRNA (guanine(26)-N2/guanine(27)-N2)-dimethyltransferase activity [GO:0160103] (molecular function) Definition: Catalysis of the reaction: guanosine(26)/guanosine(27) in tRNA + 4 S-adenosyl-L-methionine = 4 H+ + N(2)-dimethylguanosine(26)/N(2)-dimethylguanosine(27) in tRNA + 4 S-adenosyl-L-homocysteine. Sources: EC:2.1.1.215 Also known as: tRNA (guanine(26)-N(2)/guanine(27)-N(2))-dimethyltransferase activity, tRNA (guanosine(26)-N(2)/guanosine(27)-N(2))-dimethyltransferase activity Relationships: is a type of N-methyltransferase activity [GO:0008170]; is a type of tRNA (guanine) methyltransferase activity [GO:0016423]